{
  "gene": "UniProtKB:Q99594",
  "gene_name": "Transcriptional enhancer factor TEF-5",
  "gene_symbol": "TEAD3",
  "term_label": "RNA polymerase II cis-regulatory region sequence-specific DNA binding",
  "term_id": "GO:0000978"
}